{
  "gene_name": "Sin3 histone deacetylase corepressor complex component SDS3",
  "term_id": "GO:0000122",
  "term_label": "negative regulation of transcription by RNA polymerase II",
  "gene_symbol": "SUDS3",
  "gene": "UniProtKB:Q9H7L9"
}